{
  "gene_symbol": "RWDD1",
  "term_label": "Unknown cellular component",
  "gene_name": "RWD domain-containing protein 1",
  "gene": "UniProtKB:Q9H446",
  "term_id": "UNKNOWN:0003"
}